{
  "term_id": "GO:0016324",
  "gene": "UniProtKB:Q16625",
  "gene_symbol": "OCLN",
  "term_label": "apical plasma membrane",
  "gene_name": "Occludin"
}